{
  "gene_name": "Carbonic anhydrase 13",
  "gene": "UniProtKB:Q8N1Q1",
  "gene_symbol": "CA13",
  "term_id": "GO:0005829",
  "term_label": "cytosol"
}